{
  "gene_symbol": "MYH13",
  "gene_name": "Myosin-13",
  "gene": "UniProtKB:Q9UKX3",
  "term_label": "cytoplasm",
  "term_id": "GO:0005737"
}